tetrose biosynthetic process [GO:0033348] (biological process) Also known as: tetrose anabolism, tetrose biosynthesis, tetrose formation, tetrose synthesis Relationships: is a type of tetrose metabolic process [GO:0033347]; is a type of GO:0046364 Subtypes: apiose biosynthetic process [GO:0033350] Sources: GOC:mah Definition: The chemical reactions and pathways resulting in the formation of a tetrose, any monosaccharide with a chain of four carbon atoms in the molecule.